{
  "term_id": "GO:0007507",
  "gene_symbol": "TGFBR2",
  "gene": "UniProtKB:P37173",
  "term_label": "heart development",
  "gene_name": "TGF-beta receptor type-2"
}